globus pallidus development [GO:0021759] (biological process) Definition: The progression of the globus pallidus over time from its initial formation until its mature state. The globus pallidus is one of the basal ganglia involved with control of voluntary movement in the brain. Relationships: is a type of GO:0048857; is part of GO:0021536 Sources: GOC:cls, GOC:dgh, GOC:dph, GOC:jid, GO_REF:0000021 Also known as: pallidum development